{
  "term_id": "UNKNOWN:0003",
  "term_label": "Unknown cellular component",
  "gene": "UniProtKB:P0DW81",
  "gene_symbol": "MARCHF6-DT",
  "gene_name": "Poly-ADP-ribosylation-amplifying and CtIP-maintaining micropeptide"
}